telomere maintenance via telomere lengthening [GO:0010833] (biological process) Regulation: regulated by regulation of telomere maintenance via telomere lengthening [GO:1904356]; negatively regulated by negative regulation of telomere maintenance via telomere lengthening [GO:1904357]; positively regulated by positive regulation of telomere maintenance via telomere lengthening [GO:1904358] Subtypes: telomere maintenance via telomerase [GO:0007004] Sources: GOC:dph, GOC:tb Definition: Any process that contributes to the maintenance of proper telomeric length and structure by affecting and monitoring the activity of telomeric proteins and lengthening the telomeric DNA. Relationships: is_a GO:0000723